{
  "term_label": "DNA-binding transcription factor activity, RNA polymerase II-specific",
  "gene_symbol": "ZNF669",
  "gene_name": "Zinc finger protein 669",
  "term_id": "GO:0000981",
  "gene": "UniProtKB:Q96BR6"
}